{
  "gene_name": "Ras-related protein Rab-39B",
  "term_id": "GO:0003924",
  "gene_symbol": "RAB39B",
  "term_label": "GTPase activity",
  "gene": "UniProtKB:Q96DA2"
}